syncytial nuclear migration [GO:0035190] (biological process) References: PMID:8314839 Sources: GOC:bf, ISBN:0879694238 Subtypes: GO:0035191, nuclear cortical migration [GO:0035192] Definition: The directed movement of nuclei within the syncytial embryo of insects. These precise temporal and spatial patterns of nuclear movement are coordinated with mitotic divisions and are required during blastoderm formation to reposition dividing nuclei from the interior of the syncytial embryo to the cortex. Relationships: is a type of nuclear migration [GO:0007097]; is part of GO:0001700